fatty acid primary amide metabolic process [GO:0062126] (biological process) Also known as: primary fatty amide metabolic process Definition: The chemical reactions and pathways, including anabolism and catabolism, by which living organisms transform primary fatty amides. Relationships: is a type of amide metabolic process [GO:0043603]; is a type of GO:1901568 Subtypes: fatty acid primary amide biosynthetic process [GO:0062112], GO:0062127 References: PMID:11128635